{
  "term_label": "regulation of transcription by RNA polymerase II",
  "gene_name": "Zinc finger protein PLAGL2",
  "term_id": "GO:0006357",
  "gene_symbol": "PLAGL2",
  "gene": "UniProtKB:Q9UPG8"
}